{
  "term_id": "GO:0006616",
  "gene": "UniProtKB:P61619",
  "gene_symbol": "SEC61A1",
  "gene_name": "Protein transport protein Sec61 subunit alpha isoform 1",
  "term_label": "SRP-dependent cotranslational protein targeting to membrane, translocation"
}